{
  "term_id": "GO:0060337",
  "term_label": "type I interferon-mediated signaling pathway",
  "gene": "UniProtKB:P05013",
  "gene_name": "Interferon alpha-6",
  "gene_symbol": "IFNA6"
}